fluid transport [GO:0042044] (biological process) Sources: GOC:ai Relationships: is a type of GO:0006810 Subtypes: water transport [GO:0006833], epithelial fluid transport [GO:0042045] Definition: The directed movement of substances that are in liquid form in normal living conditions into, out of or within a cell, or between cells, by means of some agent such as a transporter or pore.